{
  "term_id": "GO:0019901",
  "term_label": "protein kinase binding",
  "gene_name": "Rho-related GTP-binding protein RhoC",
  "gene_symbol": "RHOC",
  "gene": "UniProtKB:P08134"
}